plastid intermembrane space [GO:0009529] (cellular component) Sources: GOC:lr Relationships: is a type of organelle envelope lumen [GO:0031970]; is part of plastid envelope [GO:0009526] Subtypes: chloroplast intermembrane space [GO:0031972], GO:0031973, cyanelle intermembrane space [GO:0036014] Also known as: plastid envelope lumen Definition: The region between the inner and outer lipid bilayers of the plastid envelope.